{
  "term_label": "heme binding",
  "gene_name": "Succinate dehydrogenase [ubiquinone] cytochrome b small subunit, mitochondrial",
  "term_id": "GO:0020037",
  "gene_symbol": "SDHD",
  "gene": "UniProtKB:O14521"
}